{
  "gene": "UniProtKB:A0A8I5QJV6",
  "gene_symbol": "A0A8I5QJV6",
  "term_id": "UNKNOWN:0001",
  "gene_name": "Uncharacterized protein",
  "term_label": "Unknown molecular function"
}